endothelial to hematopoietic transition [GO:0098508] (biological process) Relationships: is a type of cell morphogenesis [GO:0000902]; is a type of delamination [GO:0060232] Definition: The generation of hematopoietic stem cells from hemogenic endothelial cells by a process that includes tight-junction dissolution and loss of cell polarity followed by delamination from the endothelium. References: PMID:20154732, PMID:22521721